{
  "gene_name": "StAR-related lipid transfer protein 7, mitochondrial",
  "term_id": "UNKNOWN:0003",
  "gene_symbol": "STARD7",
  "gene": "UniProtKB:Q9NQZ5",
  "term_label": "Unknown cellular component"
}